{
  "gene_symbol": "SHISA2",
  "gene": "UniProtKB:Q6UWI4",
  "term_id": "GO:0040037",
  "gene_name": "Protein shisa-2 homolog",
  "term_label": "negative regulation of fibroblast growth factor receptor signaling pathway"
}